{
  "term_id": "GO:0019941",
  "gene_name": "Polyubiquitin-B",
  "gene_symbol": "UBB",
  "term_label": "modification-dependent protein catabolic process",
  "gene": "UniProtKB:P0CG47"
}